{
  "gene": "UniProtKB:Q9NS62",
  "gene_name": "Thrombospondin type-1 domain-containing protein 1",
  "gene_symbol": "THSD1",
  "term_label": "Unknown biological process",
  "term_id": "UNKNOWN:0002"
}